{
  "gene_symbol": "SELL",
  "term_label": "leukocyte tethering or rolling",
  "gene": "UniProtKB:P14151",
  "term_id": "GO:0050901",
  "gene_name": "L-selectin"
}